{
  "gene_name": "GAS2-like protein 2",
  "gene": "UniProtKB:Q8NHY3",
  "gene_symbol": "GAS2L2",
  "term_id": "GO:0001578",
  "term_label": "microtubule bundle formation"
}